{
  "gene_symbol": "THRA",
  "term_label": "nucleus",
  "term_id": "GO:0005634",
  "gene_name": "Thyroid hormone receptor alpha",
  "gene": "UniProtKB:P10827"
}